{
  "gene_symbol": "IFNA17",
  "gene_name": "Interferon alpha-17",
  "term_id": "GO:0002250",
  "term_label": "adaptive immune response",
  "gene": "UniProtKB:P01571"
}